{
  "term_label": "Unknown molecular function",
  "gene_symbol": "TUBA3FP",
  "gene": "UniProtKB:A0A994J5G1",
  "gene_name": "Tubulin alpha 3f pseudogene",
  "term_id": "UNKNOWN:0001"
}